L-histidine:histamine antiporter activity [GO:0070907] (molecular function) Sources: GOC:dh Also known as: histidine:histamine antiporter activity, histidine-histamine antiporter activity, histidine/histamine antiporter activity Definition: Catalysis of the reaction: L-histidine(out) + histamine(in) = L-histidine(in) + histamine(out). Relationships: is a type of L-histidine transmembrane transporter activity [GO:0005290]; is a type of antiporter activity [GO:0015297]; is a type of histamine transmembrane transporter activity [GO:0160173]